{
  "gene_name": "Kelch-like protein 38",
  "gene": "UniProtKB:Q2WGJ6",
  "term_label": "ubiquitin-like ligase-substrate adaptor activity",
  "gene_symbol": "KLHL38",
  "term_id": "GO:1990756"
}